{
  "gene_name": "cGMP-dependent 3',5'-cyclic phosphodiesterase",
  "term_id": "GO:0005743",
  "gene": "UniProtKB:O00408",
  "gene_symbol": "PDE2A",
  "term_label": "mitochondrial inner membrane"
}